{
  "term_id": "UNKNOWN:0001",
  "term_label": "Unknown molecular function",
  "gene_symbol": "GOLGA6C",
  "gene_name": "Golgin subfamily A member 6C",
  "gene": "UniProtKB:A6NDK9"
}